{
  "gene_name": "Cyclin-A1",
  "term_label": "G1/S transition of mitotic cell cycle",
  "term_id": "GO:0000082",
  "gene": "UniProtKB:P78396",
  "gene_symbol": "CCNA1"
}